positive regulation of brain-derived neurotrophic factor receptor signaling pathway [GO:0031550] (biological process) Sources: GOC:mah Relationships: is a type of GO:0009967; is a type of GO:0031548; positively regulates brain-derived neurotrophic factor receptor signaling pathway [GO:0031547] Also known as: positive regulation of BDNF receptor signaling pathway, positive regulation of BDNF receptor signalling pathway, positive regulation of brain-derived neurotrophic factor receptor signalling pathway, up regulation of brain-derived neurotrophic factor receptor signaling pathway, up-regulation of brain-derived neurotrophic factor receptor signaling pathway, upregulation of brain-derived neurotrophic factor receptor signaling pathway, activation of brain-derived neurotrophic factor receptor signaling pathway, stimulation of brain-derived neurotrophic factor receptor signaling pathway Definition: Any process that activates or increases the frequency, rate or extent of signaling via the brain-derived neurotrophic factor receptor signaling pathway.